{
  "gene": "UniProtKB:P52292",
  "term_id": "GO:0006607",
  "gene_name": "Importin subunit alpha-1",
  "term_label": "NLS-bearing protein import into nucleus",
  "gene_symbol": "KPNA2"
}